{
  "term_id": "GO:0006405",
  "term_label": "RNA export from nucleus",
  "gene_symbol": "NUP153",
  "gene": "UniProtKB:P49790",
  "gene_name": "Nuclear pore complex protein Nup153"
}